{
  "gene": "UniProtKB:A8MUH7",
  "gene_symbol": "PDZK1P1",
  "gene_name": "Putative PDZ domain-containing protein PDZK1P1",
  "term_id": "GO:0016324",
  "term_label": "apical plasma membrane"
}